{
  "term_id": "GO:0050821",
  "gene_symbol": "DNLZ",
  "gene": "UniProtKB:Q5SXM8",
  "gene_name": "DNL-type zinc finger protein",
  "term_label": "protein stabilization"
}